{
  "gene": "UniProtKB:Q9NRS4",
  "term_label": "serine-type peptidase activity",
  "gene_name": "Transmembrane protease serine 4",
  "gene_symbol": "TMPRSS4",
  "term_id": "GO:0008236"
}